{
  "gene_symbol": "FSCN1",
  "gene": "UniProtKB:Q16658",
  "term_label": "cytoplasm",
  "gene_name": "Fascin",
  "term_id": "GO:0005737"
}